{
  "gene": "UniProtKB:P32189",
  "gene_symbol": "GK",
  "term_label": "glycerol-3-phosphate biosynthetic process",
  "gene_name": "Glycerol kinase",
  "term_id": "GO:0046167"
}